{
  "gene_symbol": "BTG2",
  "gene_name": "Protein BTG2",
  "term_id": "GO:0005737",
  "gene": "UniProtKB:P78543",
  "term_label": "cytoplasm"
}